{
  "term_id": "UNKNOWN:0003",
  "gene_name": "Cytochrome P450 4B1",
  "gene_symbol": "CYP4B1",
  "term_label": "Unknown cellular component",
  "gene": "UniProtKB:P13584"
}